regulation of ascospore wall (1->3)-beta-D-glucan biosynthetic process [GO:0060624] (biological process) Also known as: regulation of ascospore wall 1,3-beta-D-glucan biosynthetic process, regulation of ascospore wall 1,3-beta-glucan biosynthetic process Definition: Any process that modulates the rate, frequency, or extent of ascospore wall (1->3)-beta-D-glucan biosynthetic process, the chemical reactions and pathways resulting in the formation of (1->3)-beta-D-glucans, compounds composed of glucose residues linked by (1->3)-beta-D--glucosidic bonds, found in the walls of ascospores. Subtypes: positive regulation of regulation of ascospore wall (1->3)-beta-D-glucan biosynthetic process [GO:0140748] Sources: GOC:dph, GOC:tb Relationships: is_a regulation of ascospore wall beta-glucan biosynthetic process [GO:0060622]; is a type of regulation of cell wall (1->3)-beta-D-glucan biosynthetic process [GO:0090334]; regulates ascospore wall (1->3)-beta-D-glucan biosynthetic process [GO:0034413]